{
  "term_id": "GO:0015929",
  "term_label": "hexosaminidase activity",
  "gene_name": "Hexosaminidase D",
  "gene_symbol": "HEXD",
  "gene": "UniProtKB:Q8WVB3"
}